{
  "gene_name": "Ephrin-A1",
  "term_id": "GO:0046875",
  "term_label": "ephrin receptor binding",
  "gene": "UniProtKB:P20827",
  "gene_symbol": "EFNA1"
}